central nervous system projection neuron axonogenesis [GO:0021952] (biological process) Also known as: central nervous system axon tract development Definition: Generation of a long process of a CNS neuron, that carries efferent (outgoing) action potentials from the cell body towards target cells in a different central nervous system region. Subtypes: corpus callosum morphogenesis [GO:0021540], corticospinal tract morphogenesis [GO:0021957], gracilis tract morphogenesis [GO:0021958], GO:0021959, anterior commissure morphogenesis [GO:0021960], posterior commissure morphogenesis [GO:0021961], vestibulospinal tract morphogenesis [GO:0021962], spinothalamic tract morphogenesis [GO:0021963], rubrospinal tract morphogenesis [GO:0021964], spinal cord ventral commissure morphogenesis [GO:0021965], trigeminothalamic tract morphogenesis [GO:0021974], pons reticulospinal tract morphogenesis [GO:0021975], medulla reticulospinal tract morphogenesis [GO:0021976], tectospinal tract morphogenesis [GO:0021977], tectobulbar tract morphogenesis [GO:0034429] Sources: GOC:cls, GOC:dgh, GOC:dph, GOC:jid, GO_REF:0000021 Relationships: is a type of central nervous system neuron axonogenesis [GO:0021955]